{
  "gene": "UniProtKB:Q9NQZ7",
  "term_label": "UDP phosphatase activity",
  "gene_symbol": "ENTPD7",
  "term_id": "GO:0045134",
  "gene_name": "Ectonucleoside triphosphate diphosphohydrolase 7"
}